allophanate hydrolase activity [GO:0004039] (molecular function) Definition: Catalysis of the reaction: H2O + 3 H+ + urea-1-carboxylate = 2 CO2 + 2 NH4. Sources: EC:3.5.1.54, RHEA:19029 Also known as: allophanate lyase activity, urea-1-carboxylate amidohydrolase activity Relationships: is a type of GO:0016811